{
  "term_label": "synapse",
  "gene_symbol": "CNTNAP3",
  "gene_name": "Contactin-associated protein-like 3",
  "gene": "UniProtKB:Q9BZ76",
  "term_id": "GO:0045202"
}